cell growth involved in Malpighian tubule morphogenesis [GO:0061335] (biological process) Definition: The growth of an epithelial cell dependent on cycles of endoreplication, where growth contributes to the shaping of the Malpighian tubule. References: PMID:19783135 Sources: GOC:dph, GOC:mtg_kidney_jan10 Relationships: is a type of developmental cell growth [GO:0048588]; is a type of developmental growth involved in morphogenesis [GO:0060560]; is part of GO:0007443